{
  "gene_symbol": "RANBP3L",
  "term_id": "GO:0005643",
  "gene": "UniProtKB:Q86VV4",
  "gene_name": "Ran-binding protein 3-like",
  "term_label": "nuclear pore"
}